{
  "gene_name": "TBC1 domain family member 19",
  "gene_symbol": "TBC1D19",
  "term_id": "UNKNOWN:0003",
  "gene": "UniProtKB:Q8N5T2",
  "term_label": "Unknown cellular component"
}